{
  "gene": "UniProtKB:P0DQD5",
  "term_label": "pancreatic polypeptide receptor activity",
  "gene_symbol": "NPY4R2",
  "term_id": "GO:0001602",
  "gene_name": "Neuropeptide Y receptor type 4-2"
}